{
  "gene": "UniProtKB:Q9H2Z4",
  "term_label": "RNA polymerase II cis-regulatory region sequence-specific DNA binding",
  "term_id": "GO:0000978",
  "gene_symbol": "NKX2-4",
  "gene_name": "Homeobox protein Nkx-2.4"
}